{
  "gene_name": "Paired box protein Pax-5",
  "gene_symbol": "PAX5",
  "term_id": "GO:0007399",
  "gene": "UniProtKB:Q02548",
  "term_label": "nervous system development"
}